{
  "term_label": "early endosome",
  "term_id": "GO:0005769",
  "gene": "UniProtKB:Q96C92",
  "gene_name": "Endosome-associated-trafficking regulator 1",
  "gene_symbol": "ENTR1"
}